{
  "term_label": "mitotic nuclear division",
  "gene": "UniProtKB:Q8IXV7",
  "gene_symbol": "KLHDC8B",
  "gene_name": "Kelch domain-containing protein 8B",
  "term_id": "GO:0140014"
}